regulation of trichome morphogenesis [GO:2000039] (biological process) Sources: GOC:obol Relationships: is a type of GO:0022604; is a type of GO:0045595; is a type of regulation of leaf development [GO:2000024]; regulates trichome morphogenesis [GO:0010090] Also known as: regulation of trichome cell morphogenesis during differentiation Definition: Any process that modulates the frequency, rate or extent of trichome morphogenesis.